{
  "gene_name": "Peroxisome proliferator-activated receptor delta",
  "gene": "UniProtKB:Q03181",
  "gene_symbol": "PPARD",
  "term_label": "negative regulation of inflammatory response",
  "term_id": "GO:0050728"
}